cellular response to forskolin [GO:1904322] (biological process) References: PMID:15937517 Sources: GOC:TermGenie, GO_REF:0000071 Definition: Any process that results in a change in state or activity of a cell (in terms of movement, secretion, enzyme production, gene expression, etc.) as a result of a forskolin stimulus. Relationships: is a type of cellular response to lipid [GO:0071396]; is a type of GO:0097306; is a type of cellular response to ketone [GO:1901655]; is a type of response to forskolin [GO:1904321]